type I interferon binding [GO:0019962] (MF) Relationships: is a type of interferon binding [GO:0019961] Definition: Binding to a type I interferon. Type I interferons include the interferon-alpha, beta, delta, epsilon, zeta, kappa, tau, and omega gene families. References: PMID:15546383, PMID:16681834 Sources: GOC:add, ISBN:0126896631 Also known as: type I IFN binding, interferon-alpha binding, interferon-alpha/beta binding, interferon-beta binding, interferon-delta binding, interferon-epsilon binding, interferon-kappa binding, interferon-omega binding, interferon-tau binding, interferon-zeta binding